{
  "term_id": "UNKNOWN:0002",
  "term_label": "Unknown biological process",
  "gene_symbol": "TSPY10",
  "gene_name": "Testis-specific Y-encoded protein 10",
  "gene": "UniProtKB:P0CW01"
}